{
  "gene_name": "DNA endonuclease RBBP8",
  "gene": "UniProtKB:Q99708",
  "term_label": "DNA double-strand break processing involved in repair via single-strand annealing",
  "gene_symbol": "RBBP8",
  "term_id": "GO:0010792"
}